regulation of pre-miRNA processing [GO:2000631] (biological process) Definition: Any process that modulates the frequency, rate or extent of pre-microRNA processing. Relationships: is a type of regulation of miRNA processing [GO:1903798]; regulates pre-miRNA processing [GO:0031054] Sources: GOC:dph, GOC:sl Subtypes: negative regulation of pre-miRNA processing [GO:2000632], positive regulation of pre-miRNA processing [GO:2000633] Also known as: regulation of miRNA maturation, regulation of pre-microRNA processing